{
  "gene_name": "Protein kinase C eta type",
  "term_label": "intracellular signal transduction",
  "gene": "UniProtKB:P24723",
  "gene_symbol": "PRKCH",
  "term_id": "GO:0035556"
}